{
  "gene_name": "Calcipressin-3",
  "gene_symbol": "RCAN3",
  "gene": "UniProtKB:Q9UKA8",
  "term_id": "GO:0008597",
  "term_label": "calcium-dependent protein serine/threonine phosphatase regulator activity"
}